{
  "term_id": "UNKNOWN:0002",
  "gene_name": "Olfactory receptor 4B1",
  "gene": "UniProtKB:Q8NGF8",
  "gene_symbol": "OR4B1",
  "term_label": "Unknown biological process"
}